regulation of antigen processing and presentation of peptide antigen via MHC class I [GO:0002589] (BP) Definition: Any process that modulates the frequency, rate, or extent of antigen processing and presentation of peptide antigen via MHC class I. Subtypes: GO:0002590, positive regulation of antigen processing and presentation of peptide antigen via MHC class I [GO:0002591], regulation of antigen processing and presentation of endogenous peptide antigen via MHC class I [GO:1904282] Also known as: regulation of peptide antigen processing and presentation via MHC class I Sources: GOC:add Relationships: is a type of regulation of antigen processing and presentation of peptide antigen [GO:0002583]; regulates GO:0002474